{
  "term_id": "GO:0042790",
  "gene": "UniProtKB:Q53T94",
  "gene_symbol": "TAF1B",
  "gene_name": "TATA box-binding protein-associated factor RNA polymerase I subunit B",
  "term_label": "nucleolar large rRNA transcription by RNA polymerase I"
}